regulation of chorionic trophoblast cell proliferation [GO:1901382] (biological process) Subtypes: negative regulation of chorionic trophoblast cell proliferation [GO:1901383], positive regulation of chorionic trophoblast cell proliferation [GO:1901384] Definition: Any process that modulates the frequency, rate or extent of chorionic trophoblast cell proliferation. Relationships: is a type of regulation of cell population proliferation [GO:0042127]; regulates chorionic trophoblast cell proliferation [GO:0097360] Sources: GOC:BHF, GOC:TermGenie